mesonephric duct morphogenesis [GO:0072180] (biological process) Definition: The process in which the anatomical structures of the mesonephric duct are generated and organized. A mesonephric duct is a tube drains the mesonephros. Sources: GOC:mtg_kidney_jan10 Also known as: Wolffian duct morphogenesis Relationships: is a type of mesonephric tubule morphogenesis [GO:0072171]; is a type of GO:0072178; is part of mesonephric duct development [GO:0072177] Subtypes: GO:0072181